{
  "term_id": "GO:0005634",
  "gene": "UniProtKB:Q07869",
  "gene_name": "Peroxisome proliferator-activated receptor alpha",
  "gene_symbol": "PPARA",
  "term_label": "nucleus"
}